 [go#goslim:plant:ribbon] Note: Plant GO ribbon